response to muscle inactivity involved in regulation of muscle adaptation [GO:0014877] (biological process) Subtypes: detection of muscle inactivity involved in regulation of muscle adaptation [GO:0014884], response to rest involved in regulation of muscle adaptation [GO:0014893], response to denervation involved in regulation of muscle adaptation [GO:0014894] Relationships: is a type of response to muscle inactivity [GO:0014870]; is a type of response to stimulus involved in regulation of muscle adaptation [GO:0014874] Definition: Any process that results in a change in state or activity of a cell or an organism (in terms of movement, secretion, enzyme production, gene expression, etc.) as a result of a muscle inactivity stimulus. This process occurs as part of the regulation of muscle adaptation. Sources: GOC:ef, GOC:mtg_muscle